respiratory basal cell differentiation [GO:1902691] (biological process) Relationships: is_a stem cell differentiation [GO:0048863] Also known as: airway basal cell differentiation Definition: The process in which a relatively unspecialized cell acquires the specialized features of a respiratory basal cell. Note: Changes in the lineage choice of ABCs or their undifferentiated daughters might contribute to the mucous cell hyperplasia, metaplasia or squamous metaplasia seen in many respiratory disorders References: PMID:17909629 Sources: GOC:TermGenie, GO_REF:0000086, MP:0011114